phagocytic vesicle [GO:0045335] (cellular component) Definition: A membrane-bounded intracellular vesicle that arises from the ingestion of particulate material by phagocytosis. Sources: GOC:go_curators, ISBN:0198506732 Subtypes: early phagosome [GO:0032009], phagolysosome [GO:0032010], clathrin-coated phagocytic vesicle [GO:0045336], pexophagosome [GO:1990457] Also known as: phagosome Relationships: is a type of endocytic vesicle [GO:0030139]